activated T cell proliferation [GO:0050798] (biological process) Definition: The expansion of a T cell population following activation by an antigenic stimulus. Sources: GOC:add, GOC:dph Also known as: activated T lymphocyte proliferation, activated T-cell proliferation, activated T-lymphocyte proliferation, proliferation of activated T cells Note: Note that this term refers to the proliferation of previously activated T cells; it is to be used for gene products involved in T cell proliferation following an antigenic stimulus, including both proteins internal to the T cell and external factors, such as IL-2, which specifically promote proliferation of activated T cells. Relationships: is a type of T cell proliferation [GO:0042098] Regulation: positively regulated by positive regulation of activated T cell proliferation [GO:0042104]; regulated by regulation of activated T cell proliferation [GO:0046006]; negatively regulated by negative regulation of activated T cell proliferation [GO:0046007]